negative regulation of glutamine transport [GO:2000486] (biological process) Also known as: negative regulation of L-glutamine transport Subtypes: GO:1901035 Sources: GOC:obol Relationships: is a type of negative regulation of organic acid transport [GO:0032891]; is a type of negative regulation of amino acid transport [GO:0051956]; is a type of regulation of glutamine transport [GO:2000485]; negatively regulates glutamine transport [GO:0006868] Definition: Any process that stops, prevents or reduces the frequency, rate or extent of glutamine transport.